{
  "gene_name": "B-cell antigen receptor complex-associated protein alpha chain",
  "term_id": "GO:0009897",
  "term_label": "external side of plasma membrane",
  "gene": "UniProtKB:P11912",
  "gene_symbol": "CD79A"
}